{
  "term_id": "GO:1902476",
  "gene_name": "Glycine receptor subunit alpha-3",
  "term_label": "chloride transmembrane transport",
  "gene_symbol": "GLRA3",
  "gene": "UniProtKB:O75311"
}